{
  "gene": "UniProtKB:Q86U02",
  "gene_symbol": "LINC00596",
  "term_label": "Unknown biological process",
  "gene_name": "Putative uncharacterized protein encoded by LINC00596",
  "term_id": "UNKNOWN:0002"
}